regulation of epiboly involved in gastrulation with mouth forming second [GO:1904086] (biological process) Subtypes: negative regulation of epiboly involved in gastrulation with mouth forming second [GO:1904087], GO:1904088 Relationships: is a type of GO:1905330; regulates epiboly involved in gastrulation with mouth forming second [GO:0055113] Definition: Any process that modulates the frequency, rate or extent of epiboly involved in gastrulation with mouth forming second. References: PMID:24892953 Sources: GOC:TermGenie, GO_REF:0000058